{
  "gene_name": "Zinc finger and SCAN domain-containing protein 12",
  "term_label": "DNA-binding transcription factor activity, RNA polymerase II-specific",
  "gene": "UniProtKB:O43309",
  "term_id": "GO:0000981",
  "gene_symbol": "ZSCAN12"
}